{
  "term_id": "GO:0001843",
  "gene_symbol": "VASP",
  "gene_name": "Vasodilator-stimulated phosphoprotein",
  "term_label": "neural tube closure",
  "gene": "UniProtKB:P50552"
}